N,N'-diacetylbacilliosaminyl-1-phosphate transferase activity [GO:0102334] (molecular function) Relationships: is_a phosphotransferase activity, for other substituted phosphate groups [GO:0016780] Sources: EC:2.7.8.36, GOC:pz Definition: Catalysis of the reaction: ditrans,polycis-undecaprenyl phosphate + UDP-N,N'-diacetylbacillosamine = N,N'-diacetyl-alpha-D-bacillosaminyl-diphospho-tri-trans,hepta-cis-undecaprenol + UMP.